{
  "gene_symbol": "FOXI1",
  "term_label": "anatomical structure morphogenesis",
  "term_id": "GO:0009653",
  "gene": "UniProtKB:Q12951",
  "gene_name": "Forkhead box protein I1"
}